UMP catabolic process [GO:0046050] (biological process) Definition: The chemical reactions and pathways resulting in the breakdown of UMP, uridine monophosphate. Sources: GOC:go_curators Relationships: is a type of pyrimidine ribonucleoside monophosphate catabolic process [GO:0009175]; is a type of pyrimidine ribonucleotide catabolic process [GO:0009222]; is a type of UMP metabolic process [GO:0046049] Also known as: UMP breakdown, UMP catabolism, UMP degradation